{
  "gene": "UniProtKB:O94952",
  "gene_symbol": "FBXO21",
  "term_label": "Unknown cellular component",
  "term_id": "UNKNOWN:0003",
  "gene_name": "F-box only protein 21"
}